{
  "gene": "UniProtKB:A8MXZ1",
  "term_id": "UNKNOWN:0002",
  "gene_name": "Putative protein FAM90A23",
  "gene_symbol": "FAM90A23",
  "term_label": "Unknown biological process"
}